{
  "gene_symbol": "CHRNA3",
  "term_id": "GO:0099171",
  "gene": "UniProtKB:P32297",
  "gene_name": "Neuronal acetylcholine receptor subunit alpha-3",
  "term_label": "presynaptic modulation of chemical synaptic transmission"
}